response to 3-methylcholanthrene [GO:1904681] (biological process) References: PMID:9224771 Sources: GOC:TermGenie, GOC:mr, GO_REF:0000071 Subtypes: cellular response to 3-methylcholanthrene [GO:1904682] Relationships: is a type of GO:1903165 Definition: Any process that results in a change in state or activity of a cell or an organism (in terms of movement, secretion, enzyme production, gene expression, etc.) as a result of a 3-methylcholanthrene stimulus.